fatty-acyl-CoA synthase activity [GO:0004321] (molecular function) Sources: EC:2.3.1.86 Relationships: is a type of C-acyltransferase activity [GO:0016408] Definition: Catalysis of the reaction: acetyl-CoA + n malonyl-CoA + 2n NADH + 2n NADPH + 4n H+ = a long-chain acyl-CoA + n CoA + n CO2 + 2n NAD+ + 2n NADP+. Also known as: fatty acyl CoA synthase activity, yeast fatty acid synthase activity, acyl-CoA:malonyl-CoA C-acyltransferase (decarboxylating, oxoacyl- and enoyl- reducing)